positive regulation of pseurotin A biosynthetic process [GO:1900851] (biological process) Definition: Any process that activates or increases the frequency, rate or extent of pseurotin A biosynthetic process. Also known as: up regulation of pseurotin A biosynthetic process, up-regulation of pseurotin A biosynthetic process, upregulation of pseurotin A biosynthetic process Sources: GOC:TermGenie, GOC:di Relationships: is_a positive regulation of biosynthetic process [GO:0009891]; is_a positive regulation of amide metabolic process [GO:0034250]; is a type of positive regulation of small molecule metabolic process [GO:0062013]; is a type of GO:1900849; positively regulates pseurotin A biosynthetic process [GO:1900790]